{
  "term_label": "CCR chemokine receptor binding",
  "term_id": "GO:0048020",
  "gene_name": "C-C motif chemokine 16",
  "gene": "UniProtKB:O15467",
  "gene_symbol": "CCL16"
}